{
  "gene_name": "Programmed cell death protein 5",
  "gene_symbol": "PDCD5",
  "gene": "UniProtKB:O14737",
  "term_id": "GO:0005829",
  "term_label": "cytosol"
}